{
  "term_label": "calcium ion binding",
  "term_id": "GO:0005509",
  "gene_symbol": "S100A5",
  "gene": "UniProtKB:P33763",
  "gene_name": "Protein S100-A5"
}